{
  "term_id": "GO:1990757",
  "gene": "UniProtKB:Q86Y33",
  "term_label": "ubiquitin ligase activator activity",
  "gene_name": "Cell division cycle protein 20 homolog B",
  "gene_symbol": "CDC20B"
}